{
  "gene_name": "Polyadenylate-binding protein 1",
  "gene_symbol": "PABPC1",
  "term_label": "poly(A) binding",
  "gene": "UniProtKB:P11940",
  "term_id": "GO:0008143"
}